{
  "gene": "UniProtKB:P59091",
  "term_label": "Unknown cellular component",
  "term_id": "UNKNOWN:0003",
  "gene_name": "Putative uncharacterized protein encoded by LINC00315",
  "gene_symbol": "LINC00315"
}